guanidinoacetate N-methyltransferase activity [GO:0030731] (molecular function) Definition: Catalysis of the reaction: S-adenosyl-L-methionine + guanidinoacetate = S-adenosyl-L-homocysteine + creatine + H+. Relationships: is a type of S-adenosylmethionine-dependent methyltransferase activity [GO:0008757] Also known as: GA methylpherase activity, S-adenosyl-L-methionine:N-guanidinoacetate methyltransferase activity, guanidinoacetate methyltransferase activity, guanidinoacetate transmethylase activity, guanidoacetate methyltransferase activity, methionine-guanidinoacetic transmethylase activity Sources: EC:2.1.1.2, RHEA:10656